{
  "gene_symbol": "GSDMD",
  "term_label": "phosphatidylserine binding",
  "gene_name": "Gasdermin-D",
  "term_id": "GO:0001786",
  "gene": "UniProtKB:P57764"
}